{
  "term_id": "GO:0006383",
  "gene_name": "Transcription factor IIIB 90 kDa subunit",
  "gene_symbol": "BRF1",
  "term_label": "transcription by RNA polymerase III",
  "gene": "UniProtKB:Q92994"
}